{
  "gene_symbol": "CCND1",
  "term_label": "cytoplasm",
  "gene_name": "G1_S-specific cyclin-D1",
  "term_id": "GO:0005737",
  "gene": "UniProtKB:P24385"
}